{
  "term_id": "GO:0007420",
  "term_label": "brain development",
  "gene": "UniProtKB:A6NDR6",
  "gene_name": "Putative homeobox protein Meis3-like 1",
  "gene_symbol": "MEIS3P1"
}